purine deoxyribonucleoside diphosphate biosynthetic process [GO:0009183] (biological process) Relationships: is a type of purine nucleoside diphosphate biosynthetic process [GO:0009136]; is a type of purine deoxyribonucleoside diphosphate metabolic process [GO:0009182]; is a type of GO:0009189 Sources: GOC:go_curators, ISBN:0198506732 Subtypes: GO:0006173, dGDP biosynthetic process [GO:0006185] Definition: The chemical reactions and pathways resulting in the formation of purine deoxyribonucleoside diphosphate, a compound consisting of a purine base linked to a deoxyribose sugar esterified with diphosphate on the sugar. Also known as: purine deoxyribonucleoside diphosphate anabolism, purine deoxyribonucleoside diphosphate biosynthesis, purine deoxyribonucleoside diphosphate formation, purine deoxyribonucleoside diphosphate synthesis